{
  "gene_name": "E3 ubiquitin-protein ligase RNF31",
  "gene": "UniProtKB:Q96EP0",
  "gene_symbol": "RNF31",
  "term_id": "GO:1990450",
  "term_label": "linear polyubiquitin binding"
}